{
  "gene": "UniProtKB:P37231",
  "term_label": "DNA-binding transcription repressor activity, RNA polymerase II-specific",
  "term_id": "GO:0001227",
  "gene_name": "Peroxisome proliferator-activated receptor gamma",
  "gene_symbol": "PPARG"
}